{
  "term_label": "excitatory postsynaptic potential",
  "gene_name": "Pro-FMRFamide-related neuropeptide FF",
  "term_id": "GO:0060079",
  "gene": "UniProtKB:O15130",
  "gene_symbol": "NPFF"
}